{
  "gene_symbol": "PPIAL4G",
  "term_label": "peptidyl-prolyl cis-trans isomerase activity",
  "term_id": "GO:0003755",
  "gene_name": "Peptidyl-prolyl cis-trans isomerase A-like 4G",
  "gene": "UniProtKB:P0DN37"
}